{
  "gene_symbol": "SRGAP2",
  "gene_name": "SLIT-ROBO Rho GTPase-activating protein 2",
  "gene": "UniProtKB:O75044",
  "term_label": "regulation of synapse assembly",
  "term_id": "GO:0051963"
}